{
  "gene_name": "Chymotrypsinogen B",
  "term_id": "GO:0006508",
  "term_label": "proteolysis",
  "gene_symbol": "CTRB1",
  "gene": "UniProtKB:P17538"
}